{
  "term_id": "GO:0030424",
  "gene": "UniProtKB:P49840",
  "gene_name": "Glycogen synthase kinase-3 alpha",
  "term_label": "axon",
  "gene_symbol": "GSK3A"
}